interleukin-33 production [GO:0072639] (biological process) Also known as: IL-33 production, IL33 production, NF-HEV production, C9orf26 production, IL1F11 production, interleukin-33 biosynthetic process, interleukin-33 secretion Definition: The appearance of interleukin-33 due to biosynthesis or secretion following a cellular stimulus, resulting in an increase in its intracellular or extracellular levels. Relationships: is a type of cytokine production [GO:0001816] Regulation: RO_0002211 by regulation of interleukin-33 production [GO:0150127]; negatively regulated by negative regulation of interleukin-33 production [GO:0150128]; positively regulated by positive regulation of interleukin-33 production [GO:0150129] References: PMID:29778524 Sources: GOC:BHF, GOC:mah